{
  "gene_symbol": "SCAMP5",
  "term_label": "recycling endosome membrane",
  "gene": "UniProtKB:Q8TAC9",
  "gene_name": "Secretory carrier-associated membrane protein 5",
  "term_id": "GO:0055038"
}